{
  "gene": "UniProtKB:Q9NP81",
  "term_label": "tRNA binding",
  "term_id": "GO:0000049",
  "gene_symbol": "SARS2",
  "gene_name": "Serine--tRNA ligase, mitochondrial"
}